{
  "term_label": "plasma membrane",
  "gene_name": "Lymphocyte antigen 75",
  "gene": "UniProtKB:O60449",
  "term_id": "GO:0005886",
  "gene_symbol": "LY75"
}